{
  "term_id": "GO:0005739",
  "gene_name": "Aspartate--tRNA ligase, mitochondrial",
  "gene": "UniProtKB:Q6PI48",
  "term_label": "mitochondrion",
  "gene_symbol": "DARS2"
}